ventricular zone cell fate commitment [GO:0021900] (biological process) Relationships: is a type of commitment of multipotent stem cells to neuronal lineage in forebrain [GO:0021898]; is part of forebrain neuroblast differentiation [GO:0021863] Definition: The commitment of neuroblast to become a basal progenitor cell. Basal progenitor cells are neuronal precursor cells that are committed to becoming neurons. References: PMID:16226447 Sources: GOC:cls, GOC:dgh, GOC:dph, GOC:jid, GO_REF:0000021